peptide antigen stabilization [GO:0050823] (biological process) Relationships: is a type of peptide stabilization [GO:0050822]; BFO_0000050 GO:0048002 Sources: GOC:ai Definition: Any process involved in maintaining the structure and integrity of a peptide antigen and preventing it from being degraded. Also known as: peptide antigen stabilization activity